{
  "term_label": "plasma membrane",
  "gene_name": "Orexin receptor type 2",
  "gene_symbol": "HCRTR2",
  "gene": "UniProtKB:O43614",
  "term_id": "GO:0005886"
}